{
  "gene_symbol": "CETP",
  "term_label": "phospholipid homeostasis",
  "term_id": "GO:0055091",
  "gene_name": "Cholesteryl ester transfer protein",
  "gene": "UniProtKB:P11597"
}